hydroxyproline O-galactosyltransferase activity [GO:1990714] (molecular function) References: PMID:25600942 Also known as: HPGT Definition: Catalysis of the transfer of galactose from UDP-galactose to hydroxyproline residues present in the peptide backbone. Relationships: is a type of GO:0008378